{
  "term_id": "GO:0072545",
  "gene_name": "G-protein coupled receptor 143",
  "term_label": "L-tyrosine binding",
  "gene": "UniProtKB:P51810",
  "gene_symbol": "GPR143"
}